{
  "term_id": "GO:0045214",
  "gene": "UniProtKB:Q14324",
  "term_label": "sarcomere organization",
  "gene_symbol": "MYBPC2",
  "gene_name": "Myosin-binding protein C, fast-type"
}